socket cell differentiation [GO:0090437] (biological process) Relationships: is a type of GO:0090627; is part of plant epidermis development [GO:0090558] Sources: GOC:tb Definition: The process in which a relatively unspecialized cell acquires specialized features of a socket cell, a shoot epidermal cell that surrounds a trichome and provides its support.